fructose 6-phosphate aldolase activity [GO:0097023] (molecular function) References: PMID:11120740, PMID:21290439 Sources: GOC:imk Relationships: is a type of aldehyde-lyase activity [GO:0016832] Definition: Catalysis of the reaction: D-fructose-6-phosphate = dihydroxyacetone + D-glyceraldehyde-3-phosphate.